{
  "gene": "UniProtKB:Q15329",
  "gene_symbol": "E2F5",
  "term_id": "GO:0000978",
  "term_label": "RNA polymerase II cis-regulatory region sequence-specific DNA binding",
  "gene_name": "Transcription factor E2F5"
}